{
  "gene": "UniProtKB:Q9UL36",
  "gene_symbol": "ZNF236",
  "term_label": "RNA polymerase II cis-regulatory region sequence-specific DNA binding",
  "gene_name": "Zinc finger protein 236",
  "term_id": "GO:0000978"
}